{
  "term_label": "U4/U6 x U5 tri-snRNP complex",
  "term_id": "GO:0046540",
  "gene": "UniProtKB:O43172",
  "gene_symbol": "PRPF4",
  "gene_name": "U4_U6 small nuclear ribonucleoprotein Prp4"
}